{
  "term_id": "GO:0017134",
  "gene_name": "Fibroblast growth factor receptor 2",
  "gene_symbol": "FGFR2",
  "gene": "UniProtKB:P21802",
  "term_label": "fibroblast growth factor binding"
}